{
  "term_id": "GO:0000492",
  "gene_name": "RuvB-like 1",
  "gene": "UniProtKB:Q9Y265",
  "gene_symbol": "RUVBL1",
  "term_label": "box C/D snoRNP assembly"
}